{
  "term_id": "GO:0032332",
  "gene": "UniProtKB:P48436",
  "gene_symbol": "SOX9",
  "gene_name": "Transcription factor SOX-9",
  "term_label": "positive regulation of chondrocyte differentiation"
}